{
  "term_label": "DNA-binding transcription factor activity, RNA polymerase II-specific",
  "gene_symbol": "ERF",
  "term_id": "GO:0000981",
  "gene_name": "ETS domain-containing transcription factor ERF",
  "gene": "UniProtKB:P50548"
}